methyl indole-3-acetate esterase activity [GO:0080030] (molecular function) Definition: Catalysis of the reaction: H2O + methyl (indol-3-yl)acetate = (indol-3-yl)acetate + H+ + methanol. Also known as: MeIAA esterase activity, Methyl IAA esterase activity, indole-3-Acetic acid methyl ester esterase activity Relationships: is_a GO:0052689 References: PMID:18467465 Sources: RHEA:32919